{
  "gene_symbol": "SEMA3G",
  "gene_name": "Semaphorin-3G",
  "gene": "UniProtKB:Q9NS98",
  "term_label": "chemorepellent activity",
  "term_id": "GO:0045499"
}